{
  "gene_symbol": "CAMK4",
  "gene_name": "Calcium_calmodulin-dependent protein kinase type IV",
  "term_label": "cytoplasm",
  "term_id": "GO:0005737",
  "gene": "UniProtKB:Q16566"
}